{
  "gene_name": "Keratin-associated protein 9-7",
  "term_id": "UNKNOWN:0003",
  "gene_symbol": "KRTAP9-7",
  "term_label": "Unknown cellular component",
  "gene": "UniProtKB:A8MTY7"
}